{
  "gene": "UniProtKB:Q8NEG4",
  "term_label": "Unknown cellular component",
  "gene_symbol": "FAM83F",
  "term_id": "UNKNOWN:0003",
  "gene_name": "Protein FAM83F"
}